negative regulation of oligodendrocyte differentiation [GO:0048715] (biological process) References: PMID:15139015 Sources: GOC:vp Also known as: down regulation of oligodendrocyte differentiation, down-regulation of oligodendrocyte differentiation, downregulation of oligodendrocyte differentiation, inhibition of oligodendrocyte differentiation Relationships: is a type of negative regulation of glial cell differentiation [GO:0045686]; is a type of regulation of oligodendrocyte differentiation [GO:0048713]; negatively regulates oligodendrocyte differentiation [GO:0048709] Definition: Any process that stops, prevents, or reduces the frequency, rate or extent of oligodendrocyte differentiation.